positive regulation of myeloid cell differentiation [GO:0045639] (biological process) Subtypes: positive regulation of myeloid leukocyte differentiation [GO:0002763], positive regulation of erythrocyte differentiation [GO:0045648], positive regulation of megakaryocyte differentiation [GO:0045654], positive regulation of platelet formation [GO:1905221] Relationships: is a type of positive regulation of cell differentiation [GO:0045597]; is a type of GO:0045637; positively regulates GO:0030099 Definition: Any process that activates or increases the frequency, rate or extent of myeloid cell differentiation. Sources: GOC:go_curators Also known as: up regulation of myeloid cell differentiation, up-regulation of myeloid cell differentiation, upregulation of myeloid cell differentiation, activation of myeloid cell differentiation, stimulation of myeloid cell differentiation